{
  "gene_name": "Kelch-like protein 20",
  "gene_symbol": "KLHL20",
  "term_label": "Golgi to endosome transport",
  "term_id": "GO:0006895",
  "gene": "UniProtKB:Q9Y2M5"
}